{
  "term_label": "membrane",
  "gene_name": "Sarcoplasmic_endoplasmic reticulum calcium ATPase 2",
  "term_id": "GO:0016020",
  "gene_symbol": "ATP2A2",
  "gene": "UniProtKB:P16615"
}